{
  "term_id": "GO:0005737",
  "gene_name": "Phospholipase A and acyltransferase 2",
  "gene_symbol": "PLAAT2",
  "gene": "UniProtKB:Q9NWW9",
  "term_label": "cytoplasm"
}